{
  "gene_name": "Rho-related GTP-binding protein RhoJ",
  "term_id": "GO:0019901",
  "gene": "UniProtKB:Q9H4E5",
  "gene_symbol": "RHOJ",
  "term_label": "protein kinase binding"
}